{
  "term_id": "UNKNOWN:0002",
  "gene": "UniProtKB:P0CZ25",
  "gene_name": "Uncharacterized protein DNAH10OS",
  "term_label": "Unknown biological process",
  "gene_symbol": "DNAH10OS"
}